{
  "gene_name": "Perilipin-2",
  "term_label": "lipid storage",
  "gene": "UniProtKB:Q99541",
  "gene_symbol": "PLIN2",
  "term_id": "GO:0019915"
}